{
  "term_label": "Unknown biological process",
  "term_id": "UNKNOWN:0002",
  "gene_symbol": "LCN12",
  "gene_name": "Epididymal-specific lipocalin-12",
  "gene": "UniProtKB:Q6JVE5"
}